{
  "term_id": "GO:0005634",
  "gene": "UniProtKB:P62987",
  "term_label": "nucleus",
  "gene_symbol": "UBA52",
  "gene_name": "Ubiquitin-ribosomal protein eL40 fusion protein"
}